{
  "gene_name": "Platelet-activating factor acetylhydrolase IB subunit beta",
  "gene_symbol": "PAFAH1B1",
  "term_label": "establishment of mitotic spindle orientation",
  "term_id": "GO:0000132",
  "gene": "UniProtKB:P43034"
}